{
  "term_label": "RNA polymerase II cis-regulatory region sequence-specific DNA binding",
  "gene": "UniProtKB:Q9Y5A6",
  "gene_symbol": "ZSCAN21",
  "term_id": "GO:0000978",
  "gene_name": "Zinc finger and SCAN domain-containing protein 21"
}